{
  "gene": "UniProtKB:Q68CQ7",
  "gene_symbol": "GLT8D1",
  "term_label": "Unknown molecular function",
  "term_id": "UNKNOWN:0001",
  "gene_name": "Glycosyltransferase 8 domain-containing protein 1"
}